{
  "gene_name": "Coiled-coil domain-containing protein 28B",
  "term_id": "UNKNOWN:0002",
  "term_label": "Unknown biological process",
  "gene_symbol": "CCDC28B",
  "gene": "UniProtKB:Q9BUN5"
}